{
  "gene_name": "Tumor suppressor candidate gene 1 protein",
  "gene": "UniProtKB:Q2TAM9",
  "gene_symbol": "TUSC1",
  "term_label": "Unknown molecular function",
  "term_id": "UNKNOWN:0001"
}